{
  "gene": "UniProtKB:Q96PB8",
  "gene_name": "Leucine-rich repeat-containing protein 3B",
  "term_label": "plasma membrane",
  "term_id": "GO:0005886",
  "gene_symbol": "LRRC3B"
}